{
  "term_label": "Unknown cellular component",
  "gene": "UniProtKB:A2RTX5",
  "term_id": "UNKNOWN:0003",
  "gene_symbol": "TARS3",
  "gene_name": "Threonine--tRNA ligase 2, cytoplasmic"
}